{
  "term_id": "UNKNOWN:0002",
  "gene_name": "Protein FAM43B",
  "term_label": "Unknown biological process",
  "gene": "UniProtKB:Q6ZT52",
  "gene_symbol": "FAM43B"
}